regulation of mesodermal cell fate specification [GO:0042661] (biological process) Sources: GOC:go_curators Subtypes: negative regulation of mesodermal cell fate specification [GO:0042662], regulation of axial mesodermal cell fate specification [GO:0048328], positive regulation of mesodermal cell fate specification [GO:0048337], GO:0048349, GO:0048378, regulation of intermediate mesodermal cell fate specification [GO:0048399] Relationships: is a type of regulation of cell fate specification [GO:0042659]; is a type of regulation of mesodermal cell differentiation [GO:1905770]; is a type of regulation of animal organ morphogenesis [GO:2000027]; regulates GO:0007501 Definition: Any process that modulates the frequency, rate or extent of mesoderm cell fate specification.